Z-phenylacetaldoxime biosynthetic process [GO:0046307] (biological process) Definition: The chemical reactions and pathways resulting in the formation of Z-phenylacetaldoxime, a member of the glucosinolate group of compounds. Sources: GOC:ai Also known as: Z-phenylacetaldoxime anabolism, Z-phenylacetaldoxime biosynthesis, Z-phenylacetaldoxime formation, Z-phenylacetaldoxime synthesis Relationships: is a type of biosynthetic process [GO:0009058]; is a type of aldoxime metabolic process [GO:0019330]